regulation of division septum assembly [GO:0032955] (BP) Definition: Any process that modulates the frequency, rate or extent of division septum formation. Division septum formation is the assembly and arrangement of a septum that spans the plasma membrane interface between progeny cells following cytokinesis. Subtypes: positive regulation of division septum assembly [GO:0010973], GO:0010974, regulation of mitotic division septum assembly [GO:0140279] References: PMID:19959363, PMID:21246752, PMID:22786806 Sources: GOC:mtg_cell_cycle Relationships: is a type of regulation of cell septum assembly [GO:1901891]; regulates division septum assembly [GO:0000917] Also known as: regulation of division septum formation